inulin fructotransferase (DFA-III-forming) activity [GO:0033998] (molecular function) Definition: Catalysis of the reaction: [(2->1)-beta-D-fructosyl](n) = [(2->1)-beta-D-fructosyl](n-1) + alpha-D-fructofuranose beta-D-fructofuranose 1,2':2,3'-dianhydride. This reaction is the production of alpha-D-fructofuranose beta-D-fructofuranose 1,2':2,3'-dianhydride (DFA III) by successively eliminating the diminishing (2->1)-beta-D-fructan (inulin) chain from the terminal D-fructosyl-D-fructosyl disaccharide. Sources: EC:4.2.2.18 Also known as: 2,1-beta-D-fructan lyase (alpha-D-fructofuranose-beta-D-fructofuranose-1,2':2,3'-dianhydride-forming) activity, inulase II activity, inulin D-fructosyl-D-fructosyltransferase (1,2':2,3'-dianhydride-forming) activity, inulin D-fructosyl-D-fructosyltransferase (forming alpha-D-fructofuranose beta-D-fructofuranose 1,2':2,3'-dianhydride) activity, inulin fructotransferase (DFA-III-producing) activity, inulin fructotransferase (depolymerizing) activity, inulin fructotransferase (depolymerizing, difructofuranose-1,2':2,3'-dianhydride-forming) activity, inulinase II activity Relationships: is a type of carbon-oxygen lyase activity, acting on polysaccharides [GO:0016837]